{
  "gene_name": "Apolipoprotein A-V",
  "gene_symbol": "APOA5",
  "term_label": "cholesterol transfer activity",
  "term_id": "GO:0120020",
  "gene": "UniProtKB:Q6Q788"
}